{
  "gene_name": "Probable methyltransferase-like protein 24",
  "gene": "UniProtKB:Q5JXM2",
  "term_label": "Unknown biological process",
  "gene_symbol": "METTL24",
  "term_id": "UNKNOWN:0002"
}